{
  "term_label": "spliceosomal complex",
  "gene_symbol": "TRA2B",
  "term_id": "GO:0005681",
  "gene": "UniProtKB:P62995",
  "gene_name": "Transformer-2 protein homolog beta"
}